{
  "gene": "UniProtKB:P63267",
  "gene_name": "Actin, gamma-enteric smooth muscle",
  "term_id": "GO:0015629",
  "gene_symbol": "ACTG2",
  "term_label": "actin cytoskeleton"
}